positive regulation of sodium ion transmembrane transporter activity [GO:2000651] (biological process) Definition: Any process that activates or increases the frequency, rate or extent of sodium ion transmembrane transporter activity. Relationships: is a type of positive regulation of ion transmembrane transporter activity [GO:0032414]; is a type of positive regulation of sodium ion transmembrane transport [GO:1902307]; is_a regulation of sodium ion transmembrane transporter activity [GO:2000649]; positively regulates sodium ion transmembrane transporter activity [GO:0015081] Sources: GOC:obol Subtypes: positive regulation of sodium:proton antiporter activity [GO:0032417], GO:1903408, GO:1905152 Also known as: positive regulation of sodium transporter activity